C4-dicarboxylate transport [GO:0015740] (biological process) Definition: The directed movement of a C4-dicarboxylate into, out of or within a cell, or between cells, by means of some agent such as a transporter or pore. A C4-dicarboxylate is the anion of a dicarboxylic acid that contains four carbon atoms. Sources: GOC:krc, GOC:mah Relationships: is a type of dicarboxylic acid transport [GO:0006835] Subtypes: GO:0015729, fumarate transport [GO:0015741], GO:0015743, succinate transport [GO:0015744], GO:0015810, aspartate secretion [GO:0061528]